positive regulation of synapse structural plasticity [GO:0051835] (biological process) Definition: Any process that activates, maintains or increases the frequency, rate or extent of synaptic structural plasticity. Sources: GOC:ai Also known as: up regulation of synapse structural plasticity, up-regulation of synapse structural plasticity, upregulation of synapse structural plasticity, activation of synapse structural plasticity, stimulation of synapse structural plasticity Relationships: is a type of positive regulation of cellular component organization [GO:0051130]; is a type of regulation of synapse structural plasticity [GO:0051823]